{
  "term_label": "protein transport",
  "gene_symbol": "DENND10P1",
  "gene_name": "Putative DENN domain-containing protein 10 B",
  "term_id": "GO:0015031",
  "gene": "UniProtKB:Q6NSW5"
}